{
  "term_id": "GO:0042981",
  "term_label": "regulation of apoptotic process",
  "gene_symbol": "USP17L30",
  "gene_name": "Ubiquitin carboxyl-terminal hydrolase 17-like protein 24",
  "gene": "UniProtKB:Q0WX57"
}